peptidyl-dipeptidase inhibitor activity [GO:0060422] (molecular function) Definition: Binds to and stops, prevents or reduces the activity of a peptidyl-dipeptidase. Peptidyl-dipeptidase activity catalyzes the release of C-terminal dipeptides from a polypeptide chain. Relationships: is a type of GO:0030414; RO_0002212 GO:0008241 Sources: GOC:dph, GOC:tb